{
  "term_label": "TRAMP-dependent tRNA surveillance pathway",
  "term_id": "GO:0071038",
  "gene_symbol": "EXOSC2",
  "gene": "UniProtKB:Q13868",
  "gene_name": "Exosome complex component RRP4"
}